oxidized pyrimidine nucleobase lesion DNA N-glycosylase activity [GO:0000703] (molecular function) Also known as: DNA glycosylase/AP-lyase, DNA glycosylase/beta-lyase, bifunctional DNA glycosylase, oxidized pyrimidine base lesion DNA N-glycosylase activity, endodeoxyribonuclease III, endonuclease III, endonuclease VIII activity, pyrimidine-specific oxidized base lesion DNA N-glycosylase activity References: PMID:11554296 Sources: GOC:elh Subtypes: 5-formyluracil DNA N-glycosylase activity [GO:0034042], GO:0034043 Definition: Catalysis of the removal oxidized pyrimidine bases by cleaving the N-C1' glycosidic bond between the oxidized pyrimidine and the deoxyribose sugar. The reaction involves formation of a covalent enzyme-pyrimidine base intermediate. Release of the enzyme and free base by a beta-elimination or a beta, gamma-elimination mechanism results in the cleavage of the DNA backbone 3' of the apyrimidinic (AP) site. Note: Consider also annotating to the molecular function term 'DNA-(apurinic or apyrimidinic site) lyase activity ; GO:0003906'. Relationships: is a type of oxidized base lesion DNA N-glycosylase activity [GO:0000702]